{
  "gene_name": "Small integral membrane protein 46",
  "gene": "UniProtKB:P0DQW1",
  "term_id": "UNKNOWN:0002",
  "term_label": "Unknown biological process",
  "gene_symbol": "SMIM46"
}